protoporphyrinogen IX biosynthetic process [GO:0006782] (biological process) Definition: The chemical reactions and pathways resulting in the formation of protoporphyrinogen IX. Relationships: is a type of GO:0006779; is_a protoporphyrinogen IX metabolic process [GO:0046501]; is part of GO:0006783 Subtypes: protoporphyrinogen IX biosynthetic process from glycine [GO:0019352], protoporphyrinogen IX biosynthetic process from glutamate [GO:0019353] Sources: GOC:go_curators Also known as: protoporphyrinogen IX anabolism, protoporphyrinogen IX biosynthesis, protoporphyrinogen IX formation, protoporphyrinogen IX synthesis